{
  "gene_name": "RING finger protein 214",
  "term_label": "ubiquitin-protein transferase activity",
  "gene_symbol": "RNF214",
  "term_id": "GO:0004842",
  "gene": "UniProtKB:Q8ND24"
}